{
  "term_label": "innate immune response in mucosa",
  "term_id": "GO:0002227",
  "gene": "UniProtKB:P33778",
  "gene_name": "Histone H2B type 1-B",
  "gene_symbol": "H2BC3"
}